{
  "gene_name": "Brain-derived neurotrophic factor",
  "gene": "UniProtKB:P23560",
  "gene_symbol": "BDNF",
  "term_label": "nerve growth factor receptor binding",
  "term_id": "GO:0005163"
}